{
  "gene_name": "Interleukin-3 receptor subunit alpha",
  "gene": "UniProtKB:P26951",
  "term_id": "GO:0043235",
  "gene_symbol": "IL3RA",
  "term_label": "receptor complex"
}